hydrolase activity, acting on acid sulfur-nitrogen bonds [GO:0016826] (molecular function) Definition: Catalysis of the hydrolysis of any acid sulfur-nitrogen bond. Sources: EC:3.10.-.- Also known as: hydrolase activity, acting on acid sulphur-nitrogen bonds Relationships: is a type of hydrolase activity [GO:0016787] Subtypes: N-sulfoglucosamine sulfohydrolase activity [GO:0016250], cyclamate sulfohydrolase activity [GO:0018789]